{
  "gene_name": "HERV-H_2q24.1 provirus ancestral Env polyprotein",
  "gene": "UniProtKB:Q9N2J8",
  "term_label": "Unknown cellular component",
  "gene_symbol": "Q9N2J8",
  "term_id": "UNKNOWN:0003"
}